{
  "gene": "UniProtKB:Q8WU68",
  "term_label": "mRNA splicing, via spliceosome",
  "term_id": "GO:0000398",
  "gene_name": "Splicing factor U2AF 26 kDa subunit",
  "gene_symbol": "U2AF1L4"
}